{
  "term_id": "GO:0006516",
  "gene_name": "F-box only protein 2",
  "term_label": "glycoprotein catabolic process",
  "gene": "UniProtKB:Q9UK22",
  "gene_symbol": "FBXO2"
}